subpellicular microtubule [GO:0020025] (cellular component) References: PMID:24800253 Sources: GOC:mb Definition: Singlet microtubule that lie underneath the inner membrane pellicle complex and emanate from the basal ring of the conoid. Relationships: is_a microtubule [GO:0005874]; BFO_0000050 apical complex [GO:0020007]